{
  "gene": "UniProtKB:A6NFT4",
  "gene_name": "Cilia- and flagella-associated protein 73",
  "term_label": "Unknown biological process",
  "gene_symbol": "CFAP73",
  "term_id": "UNKNOWN:0002"
}